{
  "term_id": "GO:0010975",
  "gene": "UniProtKB:Q8IU85",
  "gene_name": "Calcium_calmodulin-dependent protein kinase type 1D",
  "gene_symbol": "CAMK1D",
  "term_label": "regulation of neuron projection development"
}